{
  "gene_symbol": "CCL3L1",
  "term_label": "chemokine activity",
  "term_id": "GO:0008009",
  "gene": "UniProtKB:P16619",
  "gene_name": "C-C motif chemokine 3-like 1"
}